response to mitotic cell cycle spindle assembly checkpoint signaling [GO:0072479] (biological process) Also known as: mitotic cell cycle spindle assembly checkpoint effector process, response to signal involved in mitotic cell cycle spindle assembly checkpoint, response to Dma1-dependent checkpoint signaling, response to Dma1-dependent checkpoint signalling Subtypes: positive regulation of mitotic sister chromatid biorientation [GO:0140429], GO:1901925 Relationships: is a type of response to mitotic spindle checkpoint signaling [GO:0072476]; is a type of response to spindle assembly checkpoint signaling [GO:0072485] Sources: GOC:mtg_cell_cycle Definition: A process that occurs in response to signals generated as a result of mitotic cell cycle spindle assembly checkpoint signaling.